{
  "gene": "UniProtKB:Q6ZN54",
  "gene_name": "Differentially expressed in FDCP 8 homolog",
  "term_id": "UNKNOWN:0002",
  "gene_symbol": "DEF8",
  "term_label": "Unknown biological process"
}